plasmacytoid dendritic cell chemotaxis [GO:0002410] (biological process) Definition: The movement of a plasmacytoid dendritic cell in response to an external stimulus. Relationships: is a type of dendritic cell chemotaxis [GO:0002407] References: PMID:15159375, PMID:15814331 Sources: GOC:add